{
  "gene_name": "Scm-like with four MBT domains protein 2",
  "gene": "UniProtKB:Q5VUG0",
  "term_label": "nucleus",
  "term_id": "GO:0005634",
  "gene_symbol": "SFMBT2"
}